{
  "term_label": "maintenance of synapse structure",
  "gene": "UniProtKB:Q7Z5L3",
  "term_id": "GO:0099558",
  "gene_symbol": "C1QL2",
  "gene_name": "Complement C1q-like protein 2"
}